NMN nucleosidase activity [GO:0019160] (molecular function) Definition: Catalysis of the reaction: H2O + nicotinamide mononucleotide = D-ribose 5-phosphate + H+ + nicotinamide. Relationships: is_a hydrolase activity, hydrolyzing N-glycosyl compounds [GO:0016799] Also known as: NMN glycohydrolase activity, NMNGhase activity, NMNase activity, nicotinamide mononucleotidase activity, nicotinamide mononucleotide nucleosidase activity, nicotinamide-nucleotide phosphoribohydrolase activity Sources: EC:3.2.2.14, RHEA:23140